{
  "gene": "UniProtKB:P35558",
  "term_label": "mitochondrion",
  "gene_symbol": "PCK1",
  "term_id": "GO:0005739",
  "gene_name": "Phosphoenolpyruvate carboxykinase, cytosolic [GTP]"
}